{
  "gene": "UniProtKB:Q9BVG8",
  "term_id": "GO:0015630",
  "gene_name": "Kinesin-like protein KIFC3",
  "term_label": "microtubule cytoskeleton",
  "gene_symbol": "KIFC3"
}